{
  "gene_name": "SHC-transforming protein 2",
  "gene_symbol": "SHC2",
  "gene": "UniProtKB:P98077",
  "term_id": "GO:0007169",
  "term_label": "cell surface receptor protein tyrosine kinase signaling pathway"
}